{
  "gene_name": "Fatty acid-binding protein, adipocyte",
  "term_id": "GO:0005634",
  "gene_symbol": "FABP4",
  "term_label": "nucleus",
  "gene": "UniProtKB:P15090"
}